positive regulation of cardiac muscle cell myoblast differentiation [GO:2000700] (biological process) Sources: GOC:obol Also known as: positive regulation of myocardial precursor cell differentiation, positive regulation of cardiac myoblast differentiation Relationships: is a type of GO:0045663; is a type of positive regulation of cardioblast differentiation [GO:0051891]; is a type of regulation of cardiac muscle cell myoblast differentiation [GO:2000690]; positively regulates cardiac muscle cell myoblast differentiation [GO:0060379] Definition: Any process that activates or increases the frequency, rate or extent of cardiac muscle cell myoblast differentiation.